microtubule bundle formation involved in mitotic spindle midzone assembly [GO:1903562] (biological process) Also known as: microtubule bundle formation involved in mitotic spindle midzone formation, microtubule bundle formation involved in spindle midzone assembly involved in mitosis, microtubule bundling involved in mitotic spindle midzone formation, microtubule bundling involved in spindle midzone assembly involved in mitosis, microtubule bundling involved in spindle midzone biogenesis involved in mitosis, microtubule bundling involved in spindle midzone formation involved in mitosis, microtubule bundling involved in mitotic spindle midzone assembly Relationships: is a type of microtubule bundle formation [GO:0001578]; is_a GO:1902850; is part of mitotic spindle midzone assembly [GO:0051256] References: PMID:15647375 Sources: GOC:TermGenie, GO_REF:0000060 Definition: Any microtubule bundle formation that is involved in spindle midzone assembly involved in mitosis.